{
  "gene_symbol": "PPP1R1C",
  "term_id": "GO:0005737",
  "term_label": "cytoplasm",
  "gene_name": "Protein phosphatase 1 regulatory subunit 1C",
  "gene": "UniProtKB:Q8WVI7"
}